lipase activity [GO:0016298] (molecular function) Regulation: negatively regulated by lipase inhibitor activity [GO:0055102]; negatively regulated by negative regulation of lipase activity [GO:0060192]; positively regulated by positive regulation of lipase activity [GO:0060193]; positively regulated by GO:0060229 Sources: GOC:mah, ISBN:0198506732 Subtypes: phospholipase activity [GO:0004620], sterol ester esterase activity [GO:0004771], triacylglycerol lipase activity [GO:0004806], monoacylglycerol lipase activity [GO:0047372], GO:0047714, diacylglycerol lipase activity [GO:0120516] Definition: Catalysis of the hydrolysis of a lipid. Relationships: is a type of hydrolase activity, acting on ester bonds [GO:0016788]